{
  "term_id": "GO:0000307",
  "gene_symbol": "CDK15",
  "term_label": "cyclin-dependent protein kinase holoenzyme complex",
  "gene": "UniProtKB:Q96Q40",
  "gene_name": "Cyclin-dependent kinase 15"
}